embryonic olfactory bulb interneuron precursor migration [GO:0021831] (biological process) Definition: The directed movement of individual interneuron precursors during the embryonic development of the olfactory bulb. Relationships: is a type of substrate-independent telencephalic tangential interneuron migration [GO:0021843]; is a type of tangential migration from the subventricular zone to the olfactory bulb [GO:0022028]; is part of olfactory bulb interneuron development [GO:0021891] References: PMID:12626695 Sources: GOC:cls, GOC:dgh, GOC:dph, GOC:jid, GO_REF:0000021